{
  "term_id": "GO:0007019",
  "gene": "UniProtKB:Q86Y91",
  "term_label": "microtubule depolymerization",
  "gene_symbol": "KIF18B",
  "gene_name": "Kinesin-like protein KIF18B"
}